{
  "gene_name": "General transcription and DNA repair factor IIH helicase subunit XPD",
  "term_label": "transcription by RNA polymerase II",
  "gene_symbol": "ERCC2",
  "gene": "UniProtKB:P18074",
  "term_id": "GO:0006366"
}